low-density lipoprotein receptor complex [GO:0062136] (cellular component) Definition: A plasma membrane protein complex capable of low-density lipoprotein particle receptor activity. It may also bind xenobiotic toxins and deliver them into the cell via endocytosis. While most substrates get degraded via the endosome the receptor is recycled to the plasma membrane. It may also act as a transducer of intracellular signal pathways and often acts in corporation with other cell-surface receptors. References: PMID:26005850 Sources: GOC:bhm Relationships: is a type of GO:0062137; is a type of GO:0098797 Also known as: LDL receptor complex, LDLR complex, low-density lipoprotein particle receptor complex